SCF-YLR352W ubiquitin ligase complex [GO:0097674] (cellular component) References: PMID:19882662 Sources: GOC:jd, GOC:vw Relationships: is a type of SCF ubiquitin ligase complex [GO:0019005] Definition: An SCF ubiquitin ligase complex in which the F-box protein is YLR352W in S. cerevisiae.